{
  "gene": "UniProtKB:Q9UKK9",
  "gene_name": "ADP-sugar pyrophosphatase",
  "term_id": "GO:0005634",
  "term_label": "nucleus",
  "gene_symbol": "NUDT5"
}